cortisol secretion [GO:0043400] (biological process) Also known as: hydrocortisone secretion Definition: The regulated release of cortisol, a steroid hormone that in humans is the major circulating hormone of the cortex, or outer layer, of the adrenal gland. Relationships: is a type of GO:0015850; is a type of GO:0035933 References: PMID:11027914 Regulation: regulated by regulation of cortisol secretion [GO:0051462]; negatively regulated by GO:0051463; positively regulated by positive regulation of cortisol secretion [GO:0051464]